L-glutamine, sodium:proton antiporter activity [GO:0140830] (molecular function) Relationships: is a type of L-glutamine transmembrane transporter activity [GO:0015186]; is_a sodium:proton antiporter activity [GO:0015385]; is a type of amino acid:monoatomic cation antiporter activity [GO:0140848] References: PMID:10619430, PMID:11742981, PMID:11850497 Definition: Enables the transfer of a solute or solutes from one side of a membrane to the other according to the reaction: H+(in) + L-glutamine(out) + Na+(out) = H+(out) + L-glutamine(in) + Na+(in).